ACP phosphopantetheine attachment site binding [GO:0044620] (molecular function) Relationships: is a type of prosthetic group binding [GO:0051192] Sources: GOC:jl, GOC:vw Definition: Binding to the attachment site of the phosphopantetheine prosthetic group of an acyl carrier protein (ACP). Subtypes: acyl carrier activity [GO:0000036]